{
  "term_id": "GO:0006979",
  "gene_symbol": "PRDX4",
  "gene_name": "Peroxiredoxin-4",
  "gene": "UniProtKB:Q13162",
  "term_label": "response to oxidative stress"
}